{
  "term_id": "GO:0008104",
  "gene": "UniProtKB:Q5JQC9",
  "term_label": "intracellular protein localization",
  "gene_name": "A-kinase anchor protein 4",
  "gene_symbol": "AKAP4"
}